amylin receptor complex 1 [GO:0150056] (CC) References: PMID:22500019 Sources: GOC:aruk, GOC:bc Relationships: is a type of amylin receptor complex [GO:1903440] Also known as: AMY1 complex Definition: A G protein-coupled receptor complex that serves as a receptor for amylin polypeptide (AMY) and consists of a calcitonin receptor (CTR/CALCR) and a receptor activity-modifying protein (RAMP) 1. Amylin receptor complex 1 (AMY1) also serves as a receptor for the calcitonin related peptide (CGRP) and adrenomedullin (AM/ADM).